{
  "term_label": "Unknown molecular function",
  "gene_name": "Beta-taxilin",
  "gene_symbol": "TXLNB",
  "gene": "UniProtKB:Q8N3L3",
  "term_id": "UNKNOWN:0001"
}